transcription regulatory region RNA binding [GO:0001068] (molecular function) Definition: Binding to a RNA region within the transcript that regulates the transcription of a gene, cistron, or operon. Sources: GOC:txnOH Relationships: is_a regulatory region RNA binding [GO:0001069]